negative regulation of very-low-density lipoprotein particle clearance [GO:0010916] (biological process) Sources: GOC:BHF, GOC:dph, GOC:tb Also known as: negative regulation of VLDL clearance, negative regulation of VLDL particle clearance Definition: Any process that decreases the rate, frequency or extent of very-low-density lipoprotein particle clearance. Very-low-density lipoprotein particle clearance is the process in which a very-low-density lipoprotein particle is removed from the blood via receptor-mediated endocytosis and its constituent parts degraded. Relationships: is_a regulation of very-low-density lipoprotein particle clearance [GO:0010915]; is a type of GO:0010985; negatively regulates GO:0034447